{
  "term_label": "lysosome",
  "term_id": "GO:0005764",
  "gene": "UniProtKB:Q9H1C4",
  "gene_symbol": "UNC93B1",
  "gene_name": "Protein unc-93 homolog B1"
}